{
  "gene_name": "Ras-related protein Rab-7L1",
  "gene": "UniProtKB:O14966",
  "term_label": "endomembrane system",
  "gene_symbol": "RAB29",
  "term_id": "GO:0012505"
}